homospermidine synthase (spermidine-specific) activity [GO:0050514] (molecular function) Also known as: spermidine:putrescine 4-aminobutyltransferase (propane-1,3-diamine-forming) Sources: EC:2.5.1.45, MetaCyc:2.5.1.45-RXN Relationships: is a type of transferase activity, transferring alkyl or aryl (other than methyl) groups [GO:0016765] Definition: Catalysis of the reaction: spermidine + putrescine = sym-homospermidine + propane-1,3-diamine.